{
  "term_id": "GO:0038023",
  "gene_symbol": "FOLR2",
  "term_label": "signaling receptor activity",
  "gene_name": "Folate receptor beta",
  "gene": "UniProtKB:P14207"
}